{
  "term_id": "GO:0006891",
  "term_label": "intra-Golgi vesicle-mediated transport",
  "gene": "UniProtKB:Q5JT25",
  "gene_name": "Ras-related protein Rab-41",
  "gene_symbol": "RAB41"
}